{
  "term_label": "Unknown biological process",
  "gene_symbol": "FAM222B",
  "gene_name": "Protein FAM222B",
  "term_id": "UNKNOWN:0002",
  "gene": "UniProtKB:Q8WU58"
}